{
  "gene_symbol": "SHC3",
  "gene": "UniProtKB:Q92529",
  "term_label": "receptor tyrosine kinase binding",
  "term_id": "GO:0030971",
  "gene_name": "SHC-transforming protein 3"
}